establishment of protein localization to spindle pole body [GO:0071989] (biological process) Definition: The directed movement of a protein to a specific location at the spindle pole body. Relationships: is a type of protein localization to spindle pole body [GO:0071988]; is a type of establishment of protein localization to organelle [GO:0072594] Sources: GOC:mah Subtypes: GO:1990852 Also known as: establishment of protein localisation to spindle pole body